ommochrome metabolic process [GO:0046152] (biological process) Definition: The chemical reactions and pathways involving ommochromes, any of a large group of natural polycyclic pigments commonly found in the Arthropoda, particularly in the ommatidia of the compound eye. Sources: ISBN:0198506732 Subtypes: ommochrome biosynthetic process [GO:0006727], ommochrome catabolic process [GO:0046153] Also known as: ommochrome metabolism Relationships: is a type of eye pigment metabolic process [GO:0042441]; is_a ocellus pigment metabolic process [GO:0046158]